{
  "term_id": "GO:0005737",
  "term_label": "cytoplasm",
  "gene_symbol": "UCKL1",
  "gene_name": "Uridine-cytidine kinase-like 1",
  "gene": "UniProtKB:Q9NWZ5"
}